bis(5'-nucleosyl)-tetraphosphatase (symmetrical) activity [GO:0008803] (molecular function) Definition: Catalysis of the reaction: P(1),P(4)-bis(5'-adenosyl) tetraphosphate + H2O = 2 ADP + 2 H+. Also known as: Ap(4)A hydrolase activity, Ap4A hydrolase activity, diadenosine tetraphosphatase (symmetrical), 1-P,4-P-bis(5'-nucleosyl)-tetraphosphate nucleosidebisphosphohydrolase activity, P1,P4-bis(5'-nucleosyl)-tetraphosphate nucleosidebisphosphohydrolase activity, adenosine tetraphosphate phosphodiesterase activity, bis(5'-adenosyl) tetraphosphatase activity, diadenosine 5',5'''-P(1),P(4)-tetraphosphate pyrophosphohydrolase activity, diadenosine 5',5'''-P1,P4-tetraphosphatase activity, diadenosine 5',5'''-P1,P4-tetraphosphate pyrophosphohydrolase activity, diadenosine polyphosphate hydrolase activity, diadenosine tetraphosphate hydrolase activity, diadenosinetetraphosphatase (symmetrical) activity, dinucleosidetetraphosphatase (symmetrical) activity, dinucleosidetetraphosphate (symmetrical), symmetrical diadenosine tetraphosphate hydrolase activity Relationships: is a type of bis(5'-nucleosyl)-tetraphosphatase activity [GO:0008796] Sources: EC:3.6.1.41, RHEA:24252